reverse cholesterol transport [GO:0043691] (BP) Relationships: is a type of cholesterol transport [GO:0030301] References: PMID:7751809 Sources: GOC:ecd Definition: The directed movement of peripheral cell cholesterol, cholest-5-en-3-beta-ol, towards the liver for catabolism. Regulation: regulated by regulation of reverse cholesterol transport [GO:1903062]; negatively regulated by negative regulation of reverse cholesterol transport [GO:1903063]; positively regulated by positive regulation of reverse cholesterol transport [GO:1903064]